{
  "term_id": "GO:0003954",
  "term_label": "NADH dehydrogenase activity",
  "gene_symbol": "NDUFV2",
  "gene": "UniProtKB:P19404",
  "gene_name": "NADH dehydrogenase [ubiquinone] flavoprotein 2, mitochondrial"
}